{
  "term_label": "plasma membrane",
  "term_id": "GO:0005886",
  "gene_symbol": "CR1L",
  "gene_name": "Complement component receptor 1-like protein",
  "gene": "UniProtKB:Q2VPA4"
}